notum cell fate specification [GO:0035310] (BP) Relationships: is a type of GO:0060573; is part of wing and notum subfield formation [GO:0035309] Definition: The process in which a cell in the larval wing imaginal disc becomes capable of differentiating autonomously into a notum cell, if left in its normal environment. References: PMID:10860999